{
  "term_label": "neuropeptide signaling pathway",
  "gene": "UniProtKB:O43613",
  "gene_symbol": "HCRTR1",
  "gene_name": "Orexin_Hypocretin receptor type 1",
  "term_id": "GO:0007218"
}